cerebral cortex GABAergic interneuron migration [GO:0021853] (biological process) Definition: The migration of GABAergic interneuron precursors from the subpallium to the cerebral cortex. Relationships: is a type of interneuron migration from the subpallium to the cortex [GO:0021830]; is a type of interneuron migration [GO:1904936]; is part of cerebral cortex GABAergic interneuron development [GO:0021894] References: PMID:12626695 Sources: GOC:cls, GOC:dgh, GOC:dph, GOC:jid, GO_REF:0000021